catalytic activity, acting on a protein [GO:0140096] (molecular function) Sources: GOC:molecular_function_refactoring, GOC:pdt Relationships: is a type of catalytic activity [GO:0003824] Subtypes: peptidyltransferase activity [GO:0000048], GO:0003755, protein disulfide isomerase activity [GO:0003756], GO:0003810, GO:0003875, arginyl-tRNA--protein transferase activity [GO:0004057], biotin--[biotin carboxyl-carrier protein] ligase activity [GO:0004077], dihydrolipoyllysine-residue succinyltransferase activity [GO:0004149], dolichyl-phosphate-mannose-protein mannosyltransferase activity [GO:0004169], GO:0004408, peptidylamidoglycolate lyase activity [GO:0004598], polypeptide N-acetylgalactosaminyltransferase activity [GO:0004653], protein kinase activity [GO:0004672], protein-lysine 6-oxidase activity [GO:0004720], GO:0004721, GO:0004742, tubulin-tyrosine ligase activity [GO:0004835], peptide-methionine (S)-S-oxide reductase activity [GO:0008113], peptidase activity [GO:0008233], GO:0008276, protein prenyltransferase activity [GO:0008318], GO:0008474, procollagen-lysine 5-dioxygenase activity [GO:0008475], protein-tyrosine sulfotransferase activity [GO:0008476], GO:0008568, ubiquitin-like modifier activating enzyme activity [GO:0008641], [acyl-carrier-protein] phosphodiesterase activity [GO:0008770], [protein-PII] uridylyltransferase activity [GO:0008773], leucyl-tRNA--protein transferase activity [GO:0008914], GO:0008961, protein-disulfide reductase activity [GO:0015035], protein N-acetylglucosaminyltransferase activity [GO:0016262], glutaminyl-peptide cyclotransferase activity [GO:0016603], lipoate-protein ligase activity [GO:0016979], peptidyl-lysine N6-myristoyltransferase activity [GO:0018030], peptidyl-lysine N6-palmitoyltransferase activity [GO:0018031], deoxyhypusine monooxygenase activity [GO:0019135], protein-cysteine S-acyltransferase activity [GO:0019707], protein-phosphatidylethanolamide deconjugating activity [GO:0019786], ubiquitin-like protein transferase activity [GO:0019787], protein xylosyltransferase activity [GO:0030158], peptidyl-proline dioxygenase activity [GO:0031543], GO:0033558, peptide-methionine (R)-S-oxide reductase activity [GO:0033743], lipoyl(octanoyl) transferase activity [GO:0033819], procollagen glucosyltransferase activity [GO:0033823], Skp1-protein-hydroxyproline N-acetylglucosaminyltransferase activity [GO:0033830], peptidyl-cysteine S-nitrosylase activity [GO:0035605], GO:0036054, peptidyl-histidine dioxygenase activity [GO:0036139], [protein]-asparagine 3-dioxygenase activity [GO:0036140], protein deglycase activity [GO:0036524], protein adenylylhydrolase activity [GO:0044603], GO:0046922, GO:0047187, alpha-1,4-glucan-protein synthase (ADP-forming) activity [GO:0047211], [glutamine synthetase]-adenylyl-L-tyrosine phosphorylase activity [GO:0047388], GO:0047402, procollagen galactosyltransferase activity [GO:0050211], protein-glutamine glutaminase activity [GO:0050568], protein methylesterase activity [GO:0051723], protein-lysine lysyltransferase activity [GO:0052868], GO:0061607, microtubule plus end polymerase [GO:0061863], peptidyl-aspartic acid 3-dioxygenase activity [GO:0062101], GO:0070735, protein-glutamic acid ligase activity [GO:0070739], protein-N-terminal glutamine amidohydrolase activity [GO:0070773], GO:0070815, protein O-acetylglucosaminyltransferase activity [GO:0097363], protein-ribulosamine 3-kinase activity [GO:0102193], protein-fructosamine 3-kinase activity [GO:0102194], [protein]-3-O-(N-acetyl-D-glucosaminyl)-L-serine/L-threonine O-N-acetyl-alpha-D-glucosaminase activity [GO:0102571], GO:0103039, peptidyl-lysine 3-dioxygenase activity [GO:0106155], GO:0106156, peptidyl-arginine 3-dioxygenase activity [GO:0106157], catalytic activity, acting on a glycoprotein [GO:0140103], protein N-acyltransferase activity [GO:0140186], ADP-ribosylserine hydrolase activity [GO:0140292], ADP-ribosylglutamate hydrolase activity [GO:0140293], GO:0140457, ATP-dependent histone chaperone activity [GO:0140674], GO:0140740, cholesterol-protein transferase activity [GO:0140853], histone modifying activity [GO:0140993], RNA polymerase II CTD heptapeptide repeat modifying activity [GO:0140994], protein-glutathione oxidoreductase (glutathione) activity [GO:0141049], peptide lactyltransferase (ATP-dependent) activity [GO:0141207], GO:0141218, GO:0160216, GO:0160260, NAD+-protein mono-ADP-ribosyltransferase activity [GO:1990404] Definition: Catalytic activity that acts to modify a protein.